{
  "term_label": "actin filament",
  "gene": "UniProtKB:P67936",
  "gene_symbol": "TPM4",
  "term_id": "GO:0005884",
  "gene_name": "Tropomyosin alpha-4 chain"
}